{
  "term_id": "GO:0005886",
  "term_label": "plasma membrane",
  "gene_name": "Ephrin-A1",
  "gene_symbol": "EFNA1",
  "gene": "UniProtKB:P20827"
}